{
  "gene": "UniProtKB:Q9ULX6",
  "term_label": "nuclear matrix",
  "term_id": "GO:0016363",
  "gene_name": "A-kinase anchor protein 8-like",
  "gene_symbol": "AKAP8L"
}